{
  "gene_symbol": "TNIK",
  "gene_name": "TRAF2 and NCK-interacting protein kinase",
  "gene": "UniProtKB:Q9UKE5",
  "term_label": "neuron projection morphogenesis",
  "term_id": "GO:0048812"
}